protein-arginine omega-N symmetric methyltransferase activity [GO:0035243] (molecular function) Note: Note that type II protein arginine N-methyltransferase enzymes possess 'protein-arginine omega-N monomethyltransferase activity ; GO:0035241' and 'protein-arginine omega-N symmetric methyltransferase activity ; GO:0035243'. Also known as: protein arginine omega-N symmetric methylase activity, protein arginine omega-N symmetric methyltransferase activity, S-adenosyl-L-methionine:[protein]-L-arginine N-methyltransferase ([protein]-Nomega,Nomega'-dimethyl-L-arginine-forming), type II PRMT activity, type II protein arginine methyltransferase activity Definition: Catalysis of the addition of a second methyl group to methylated peptidyl-arginine. Methylation is on the terminal nitrogen (omega nitrogen) residue that is not already methylated, resulting in symmetrical peptidyl-N(omega),N'(omega)-dimethyled arginine residues. Relationships: is a type of protein-arginine N-methyltransferase activity [GO:0016274] References: PMID:14705965 Sources: EC:2.1.1.320, RESID:AA0067, RESID:AA0069